nicotinate riboside kinase activity [GO:0061769] (molecular function) Relationships: is a type of kinase activity [GO:0016301]; is a type of GO:0016773 Also known as: nicotinic acid riboside kinase activity, ribosylnicotinate kinase activity, ribosylnicotinic acid kinase activity References: PMID:17914902 Sources: RHEA:25568 Definition: Catalysis of the reaction: N-ribosylnicotinate + ATP = ADP + 2 H+ + nicotinate mononucleotide.